succinyl-CoA:3-oxo-acid CoA-transferase activity [GO:0008260] (molecular function) Definition: Catalysis of the reaction: succinyl-CoA + a 3-oxo acid = succinate + a 3-oxo-acyl-CoA. References: PMID:10964512, PMID:8844009 Sources: GOC:vw, RHEA:24564 Relationships: is a type of GO:0008410 Also known as: 3-oxoacid CoA-transferase activity, Succinyl-CoA:3-ketoacid-CoA transferase, 3-oxo-CoA transferase activity, 3-oxoacid CoA dehydrogenase activity, 3-oxoacid coenzyme A-transferase activity, acetoacetate succinyl-CoA transferase activity, acetoacetyl coenzyme A-succinic thiophorase activity, succinyl coenzyme A-acetoacetyl coenzyme A-transferase activity, succinyl-CoA 3-ketoacid-CoA transferase activity, succinyl-CoA transferase activity